{
  "term_id": "GO:0003700",
  "gene": "UniProtKB:B7ZLF3",
  "gene_name": "C2H2-type domain-containing protein",
  "gene_symbol": "LOC728743",
  "term_label": "DNA-binding transcription factor activity"
}